{
  "gene": "UniProtKB:Q9Y6I8",
  "term_label": "Unknown molecular function",
  "term_id": "UNKNOWN:0001",
  "gene_name": "Peroxisomal membrane protein 4",
  "gene_symbol": "PXMP4"
}